{
  "term_id": "GO:0098609",
  "gene_symbol": "CDHR5",
  "gene": "UniProtKB:Q9HBB8",
  "gene_name": "Cadherin-related family member 5",
  "term_label": "cell-cell adhesion"
}